{
  "gene": "UniProtKB:P38435",
  "term_label": "gamma-glutamyl carboxylase activity",
  "gene_name": "Vitamin K-dependent gamma-carboxylase",
  "gene_symbol": "GGCX",
  "term_id": "GO:0008488"
}